{
  "gene_symbol": "KIAA0513",
  "term_label": "Unknown biological process",
  "gene": "UniProtKB:O60268",
  "term_id": "UNKNOWN:0002",
  "gene_name": "Uncharacterized protein KIAA0513"
}